animal gross anatomical part developmental process [GO:0160108] (biological process) Sources: GOC:pg Relationships: is a type of GO:0032502 Definition: Any developmental process whose specific outcome is the progression of a gross anatomical part of an animal from an initial immature state, to a later, more mature state. Also known as: animal development